{
  "gene_name": "Inactive tyrosine-protein kinase 7",
  "gene_symbol": "PTK7",
  "gene": "UniProtKB:Q13308",
  "term_id": "GO:0005886",
  "term_label": "plasma membrane"
}